modified amino acid binding [GO:0072341] (molecular function) Also known as: amino acid derivative binding Sources: GOC:mah Definition: Binding to a modified amino acid. Subtypes: phosphatidylserine binding [GO:0001786], folic acid binding [GO:0005542], GO:0031177, 3-sulfino-L-alanine binding [GO:0036127], GO:0043295, dihydrofolic acid binding [GO:0051871], L-DOPA binding [GO:0072544] Relationships: is a type of binding [GO:0005488]